{
  "term_label": "Unknown cellular component",
  "gene_symbol": "SH3BGR",
  "term_id": "UNKNOWN:0003",
  "gene_name": "SH3 domain-binding glutamic acid-rich protein",
  "gene": "UniProtKB:P55822"
}